CERF complex [GO:0090537] (cellular component) Relationships: is a type of GO:0031010 Sources: GOC:krc Definition: An ISWI complex that contains an ATPase subunit of the ISWI family (specifically SNF2L in mammals, which contain two ISWI homologs) and a CECR2 homolog. In mammals, CERF is involved in regulation of transcription from RNA polymerase II promoters.